negative regulation of VCP-NPL4-UFD1 AAA ATPase complex assembly [GO:1904240] (biological process) Definition: Any process that stops, prevents or reduces the frequency, rate or extent of VCP-NPL4-UFD1 AAA ATPase complex assembly. Also known as: down regulation of VCP-NPL4-UFD1 AAA ATPase complex assembly, down regulation of VCP-NPL4-UFD1 AAA ATPase complex formation, down regulation of p97-Ufd1-Npl4 complex assembly, down regulation of p97-Ufd1-Npl4 complex formation, down-regulation of VCP-NPL4-UFD1 AAA ATPase complex assembly, down-regulation of VCP-NPL4-UFD1 AAA ATPase complex formation, down-regulation of p97-Ufd1-Npl4 complex assembly, down-regulation of p97-Ufd1-Npl4 complex formation, downregulation of VCP-NPL4-UFD1 AAA ATPase complex assembly, downregulation of VCP-NPL4-UFD1 AAA ATPase complex formation, downregulation of p97-Ufd1-Npl4 complex assembly, downregulation of p97-Ufd1-Npl4 complex formation, negative regulation of VCP-NPL4-UFD1 AAA ATPase complex formation, negative regulation of p97-Ufd1-Npl4 complex assembly, negative regulation of p97-Ufd1-Npl4 complex formation, down regulation of Cdc48p-Npl4p-Ufd1p AAA ATPase complex assembly, down regulation of Cdc48p-Npl4p-Ufd1p AAA ATPase complex formation, down-regulation of Cdc48p-Npl4p-Ufd1p AAA ATPase complex assembly, down-regulation of Cdc48p-Npl4p-Ufd1p AAA ATPase complex formation, downregulation of Cdc48p-Npl4p-Ufd1p AAA ATPase complex assembly, downregulation of Cdc48p-Npl4p-Ufd1p AAA ATPase complex formation, inhibition of Cdc48p-Npl4p-Ufd1p AAA ATPase complex assembly, inhibition of Cdc48p-Npl4p-Ufd1p AAA ATPase complex formation, inhibition of VCP-NPL4-UFD1 AAA ATPase complex assembly, inhibition of VCP-NPL4-UFD1 AAA ATPase complex formation, inhibition of p97-Ufd1-Npl4 complex assembly, inhibition of p97-Ufd1-Npl4 complex formation, negative regulation of Cdc48p-Npl4p-Ufd1p AAA ATPase complex assembly, negative regulation of Cdc48p-Npl4p-Ufd1p AAA ATPase complex formation References: PMID:17000876 Sources: GOC:PARL, GOC:TermGenie, GOC:bf, GO_REF:0000058 Relationships: is a type of negative regulation of protein-containing complex assembly [GO:0031333]; is a type of GO:1904239; negatively regulates VCP-NPL4-UFD1 AAA ATPase complex assembly [GO:1904210]